positive regulation of mating-type specific transcription, DNA-templated [GO:0045895] (biological process) Also known as: positive regulation of mating-type specific transcription, DNA-dependent, up regulation of transcription, mating-type specific, up-regulation of transcription, mating-type specific, upregulation of transcription, mating-type specific, activation of transcription, mating-type specific, stimulation of transcription, mating-type specific Relationships: is a type of GO:0007532; is a type of GO:0045893 Sources: GOC:go_curators, GOC:txnOH Definition: Any mating-type specific process that activates or increases the rate of cellular DNA-templated transcription.